{
  "term_id": "UNKNOWN:0001",
  "gene": "UniProtKB:Q9UHQ7",
  "term_label": "Unknown molecular function",
  "gene_symbol": "TCEAL9",
  "gene_name": "Transcription elongation factor A protein-like 9"
}